positive regulation of transcription by RNA polymerase III [GO:0045945] (biological process) Sources: GOC:go_curators, GOC:txnOH Relationships: is a type of regulation of transcription by RNA polymerase III [GO:0006359]; is a type of positive regulation of DNA-templated transcription [GO:0045893]; positively regulates transcription by RNA polymerase III [GO:0006383] Definition: Any process that activates or increases the frequency, rate or extent of transcription mediated by RNA polymerase III. Also known as: positive regulation of transcription from Pol III promoter, positive regulation of transcription from RNA polymerase III promoter, up regulation of transcription from RNA polymerase III promoter, up-regulation of transcription from RNA polymerase III promoter, upregulation of transcription from RNA polymerase III promoter, activation of transcription from RNA polymerase III promoter, stimulation of transcription from RNA polymerase III promoter